{
  "term_id": "UNKNOWN:0002",
  "gene_name": "Leucine-rich repeat-containing protein 3B",
  "gene_symbol": "LRRC3B",
  "gene": "UniProtKB:Q96PB8",
  "term_label": "Unknown biological process"
}